{
  "gene_symbol": "RPS6KB1",
  "term_label": "cytoplasm",
  "term_id": "GO:0005737",
  "gene_name": "Ribosomal protein S6 kinase beta-1",
  "gene": "UniProtKB:P23443"
}